{
  "gene_name": "Zinc finger BED domain-containing protein 3",
  "gene": "UniProtKB:Q96IU2",
  "gene_symbol": "ZBED3",
  "term_label": "positive regulation of transcription by RNA polymerase II",
  "term_id": "GO:0045944"
}